oleic acid binding [GO:0070538] (molecular function) Sources: GOC:lp, GOC:mah Relationships: is a type of long-chain fatty acid binding [GO:0036041] Definition: Binding to oleic acid, the 18-carbon monounsaturated fatty acid (9Z)-octadec-9-enoic acid.